{
  "gene": "UniProtKB:Q6P4R8",
  "gene_symbol": "NFRKB",
  "gene_name": "Nuclear factor related to kappa-B-binding protein",
  "term_label": "Unknown cellular component",
  "term_id": "UNKNOWN:0003"
}